{
  "gene": "UniProtKB:Q9UNH6",
  "term_label": "Unknown molecular function",
  "term_id": "UNKNOWN:0001",
  "gene_name": "Sorting nexin-7",
  "gene_symbol": "SNX7"
}